1,2-dichloroethane catabolic process [GO:0019260] (biological process) Also known as: 1,2-dichloroethane breakdown, 1,2-dichloroethane catabolism, 1,2-dichloroethane degradation Sources: GOC:go_curators Relationships: is a type of halogenated hydrocarbon catabolic process [GO:0042206] Definition: The chemical reactions and pathways resulting in the breakdown of 1,2-dichloroethane, a major commodity chemical used, for example, in the manufacture of vinyl chloride.